{
  "gene": "UniProtKB:Q8WWM1",
  "term_id": "UNKNOWN:0003",
  "gene_name": "X antigen family member 5",
  "gene_symbol": "XAGE5",
  "term_label": "Unknown cellular component"
}